{
  "gene": "UniProtKB:P07451",
  "term_id": "GO:0005737",
  "term_label": "cytoplasm",
  "gene_name": "Carbonic anhydrase 3",
  "gene_symbol": "CA3"
}